pituitary adenylate cyclase-activating polypeptide receptor binding [GO:0031858] (molecular function) Relationships: is a type of neuropeptide receptor binding [GO:0071855] Also known as: PACAP receptor binding, pituitary adenylate cyclase activating peptide receptor binding, pituitary adenylate cyclase-activating peptide receptor ligand Definition: Binding to a pituitary adenylate cyclase-activating polypeptide receptor. Sources: GOC:mah, GOC:nln